{
  "term_label": "vasculogenesis",
  "gene_symbol": "EGFL8",
  "gene": "UniProtKB:Q99944",
  "term_id": "GO:0001570",
  "gene_name": "Epidermal growth factor-like protein 8"
}